{
  "gene_name": "Stromal cell-derived factor 2-like protein 1",
  "gene": "UniProtKB:Q9HCN8",
  "gene_symbol": "SDF2L1",
  "term_label": "Unknown molecular function",
  "term_id": "UNKNOWN:0001"
}